{
  "gene": "UniProtKB:Q9H339",
  "term_id": "GO:0004984",
  "term_label": "olfactory receptor activity",
  "gene_name": "Olfactory receptor 51B5",
  "gene_symbol": "OR51B5"
}